{
  "gene_symbol": "KCNH2",
  "term_id": "GO:0005242",
  "gene": "UniProtKB:Q12809",
  "term_label": "inward rectifier potassium channel activity",
  "gene_name": "Potassium voltage-gated channel subfamily H member 2"
}